{
  "gene_name": "Multidrug resistance-associated protein 1",
  "gene": "UniProtKB:P33527",
  "term_id": "GO:0034634",
  "gene_symbol": "ABCC1",
  "term_label": "glutathione transmembrane transporter activity"
}